{
  "term_id": "GO:0005802",
  "term_label": "trans-Golgi network",
  "gene_name": "Carbohydrate sulfotransferase 4",
  "gene_symbol": "CHST4",
  "gene": "UniProtKB:Q8NCG5"
}